{
  "gene_symbol": "SLC4A1AP",
  "term_label": "Unknown biological process",
  "term_id": "UNKNOWN:0002",
  "gene_name": "Kanadaptin",
  "gene": "UniProtKB:Q9BWU0"
}